microglial cell activation [GO:0001774] (biological process) References: PMID:10626665, PMID:10695728, PMID:12580336, PMID:9893949 Sources: GOC:mgi_curators Relationships: is a type of leukocyte activation involved in inflammatory response [GO:0002269]; is a type of macrophage activation [GO:0042116]; is a type of GO:0061900 Subtypes: GO:0002282 Definition: The change in morphology and behavior of a microglial cell resulting from exposure to a cytokine, chemokine, cellular ligand, or soluble factor. Regulation: regulated by regulation of microglial cell activation [GO:1903978]; negatively regulated by negative regulation of microglial cell activation [GO:1903979]; positively regulated by GO:1903980